cAMP receptor activity [GO:0001646] (MF) Sources: GOC:pg Also known as: class E G protein coupled receptor, class E G-protein coupled receptor, class E GPCR, 3',5' cAMP receptor activity, 3',5'-cAMP receptor activity, adenosine 3',5'-cyclophosphate receptor activity, cyclic AMP receptor activity Relationships: is a type of G protein-coupled purinergic nucleotide receptor activity [GO:0045028]; has part cAMP binding [GO:0030552] Definition: Combining with cAMP (cyclic AMP, adenosine 3',5'-cyclophosphate) and transmitting the signal from one side of the membrane to the other to initiate a change in cell activity.